{
  "term_label": "cell adhesion",
  "gene": "UniProtKB:O76076",
  "term_id": "GO:0007155",
  "gene_name": "CCN family member 5",
  "gene_symbol": "CCN5"
}